{
  "gene": "UniProtKB:Q8NGJ7",
  "term_id": "GO:0005886",
  "gene_name": "Olfactory receptor 51A2",
  "term_label": "plasma membrane",
  "gene_symbol": "OR51A2"
}